{
  "term_label": "Unknown cellular component",
  "term_id": "UNKNOWN:0003",
  "gene": "UniProtKB:Q6L8H1",
  "gene_symbol": "KRTAP5-4",
  "gene_name": "Keratin-associated protein 5-4"
}